{
  "gene_symbol": "PLA2G10",
  "term_id": "GO:0046470",
  "gene": "UniProtKB:O15496",
  "term_label": "phosphatidylcholine metabolic process",
  "gene_name": "Group 10 secretory phospholipase A2"
}